{
  "term_id": "GO:0019901",
  "term_label": "protein kinase binding",
  "gene_symbol": "HSP90B2P",
  "gene_name": "Putative endoplasmin-like protein",
  "gene": "UniProtKB:Q58FF3"
}